branching involved in pancreas morphogenesis [GO:0061114] (biological process) Sources: GOC:dph Definition: The process in which the branches of the pancreas are generated and organized. Subtypes: GO:0061130 Relationships: is a type of morphogenesis of a branching epithelium [GO:0061138]; BFO_0000050 GO:0061113